cytoplasmic polyadenylation-dependent rRNA catabolic process [GO:0035760] (biological process) Definition: The chemical reactions and pathways occurring in the cytoplasm and resulting in the breakdown of a ribosomal RNA (rRNA) molecule, initiated by the enzymatic addition of a sequence of adenylyl residues (polyadenylation) at the 3' end the target rRNA truncated degradation intermediate. Relationships: is a type of rRNA catabolic process [GO:0016075]; is a type of GO:0043634; is a type of GO:0180018 Also known as: cytoplasmic poly(A)-dependent rRNA catabolic process References: PMID:20368444